{
  "gene_symbol": "SPTBN5",
  "gene_name": "Spectrin beta chain, non-erythrocytic 5",
  "term_id": "GO:0030864",
  "gene": "UniProtKB:Q9NRC6",
  "term_label": "cortical actin cytoskeleton"
}